{
  "gene": "UniProtKB:Q8WTR7",
  "gene_name": "Zinc finger protein 473",
  "term_id": "GO:0000122",
  "term_label": "negative regulation of transcription by RNA polymerase II",
  "gene_symbol": "ZNF473"
}